SWI/SNF superfamily-type complex [GO:0070603] (cellular component) Relationships: is a type of nuclear protein-containing complex [GO:0140513]; is a type of ATPase complex [GO:1904949]; is part of chromatin [GO:0000785] Subtypes: SWI/SNF complex [GO:0016514], RSC-type complex [GO:0016586], ISWI-type complex [GO:0031010], GO:0035060, npBAF complex [GO:0071564], GO:0071565, CHD-type complex [GO:0090545], INO80-type complex [GO:0097346], B-WICH complex [GO:0110016], mBAF complex [GO:0140091], GO:0140092, esBAF complex [GO:0140093], GBAF complex [GO:0140288] References: PMID:16155938 Sources: GOC:bhm, GOC:krc, GOC:mah Also known as: BAF-type complex, SWI-SNF-type complex, SWI-SNF global transcription activator complex, SWI/SNF-type complex, SWI2/SNF2 superfamily ATP-dependent chromatin remodeling complex Definition: A protein complex that contains an ortholog of the Saccharomyces ATPase Swi2/Snf2 as one of the catalytic subunit components (ATPase) and mediates assembly of nucleosomes, changes to the spacing or structure of nucleosomes, or some combination of those activities in a manner that requires ATP.